{
  "term_id": "GO:0005615",
  "gene_symbol": "IFNA17",
  "term_label": "extracellular space",
  "gene_name": "Interferon alpha-17",
  "gene": "UniProtKB:P01571"
}